anatomical structure regression [GO:0060033] (biological process) Relationships: is_a developmental process [GO:0032502]; is part of anatomical structure morphogenesis [GO:0009653] Also known as: histolysis, tissue death Subtypes: GO:0001880, GO:0035069, salivary gland histolysis [GO:0035070], notochord regression [GO:0060032], mammary gland duct regression in males [GO:0060641], GO:1990384 Definition: The developmental process in which an anatomical structure is destroyed as a part of its normal progression. Sources: GOC:dph